{
  "gene_name": "Vacuolar protein sorting-associated protein 18 homolog",
  "gene": "UniProtKB:Q9P253",
  "term_label": "endosome organization",
  "gene_symbol": "VPS18",
  "term_id": "GO:0007032"
}